{
  "term_id": "GO:0003875",
  "gene": "UniProtKB:P54922",
  "gene_symbol": "ADPRH",
  "term_label": "ADP-ribosylarginine hydrolase activity",
  "gene_name": "ADP-ribosylhydrolase ARH1"
}